negative regulation of mitotic DNA replication initiation from late origin [GO:0101018] (biological process) Also known as: negative regulation of late replication origin firing Definition: Any process that stops, prevents or reduces the frequency, rate or extent of firing from a late origin of replication involved in mitotic DNA replication. Relationships: is a type of regulation of mitotic DNA replication initiation from late origin [GO:0101017]; is a type of GO:1903467 References: PMID:26436827